{
  "gene_name": "Flotillin-1",
  "term_id": "GO:0072659",
  "gene_symbol": "FLOT1",
  "term_label": "protein localization to plasma membrane",
  "gene": "UniProtKB:O75955"
}